{
  "gene_name": "Zinc finger protein 430",
  "term_id": "GO:0006355",
  "gene": "UniProtKB:Q9H8G1",
  "gene_symbol": "ZNF430",
  "term_label": "regulation of DNA-templated transcription"
}